{
  "gene": "UniProtKB:O95363",
  "gene_symbol": "FARS2",
  "term_id": "GO:0004826",
  "gene_name": "Phenylalanine--tRNA ligase, mitochondrial",
  "term_label": "phenylalanine-tRNA ligase activity"
}